{
  "term_label": "regulation of transcription by RNA polymerase II",
  "gene": "UniProtKB:Q9Y467",
  "gene_name": "Sal-like protein 2",
  "term_id": "GO:0006357",
  "gene_symbol": "SALL2"
}